{
  "gene": "UniProtKB:Q9P2W3",
  "term_id": "GO:0005834",
  "gene_name": "Guanine nucleotide-binding protein G(I)_G(S)_G(O) subunit gamma-13",
  "term_label": "heterotrimeric G-protein complex",
  "gene_symbol": "GNG13"
}